{
  "gene": "UniProtKB:O75679",
  "gene_symbol": "RFPL3",
  "term_label": "ubiquitin protein ligase activity",
  "term_id": "GO:0061630",
  "gene_name": "Ret finger protein-like 3"
}